{
  "term_label": "lipid metabolic process",
  "term_id": "GO:0006629",
  "gene": "UniProtKB:Q9BTV4",
  "gene_name": "Transmembrane protein 43",
  "gene_symbol": "TMEM43"
}